{
  "gene_symbol": "IGKV4-1",
  "term_label": "Unknown molecular function",
  "gene": "UniProtKB:P06312",
  "term_id": "UNKNOWN:0001",
  "gene_name": "Immunoglobulin kappa variable 4-1"
}